negative regulation of sclerotium development [GO:1901923] (biological process) Relationships: is a type of GO:0051093; is a type of regulation of sclerotium development [GO:1901922]; negatively regulates sclerotium development [GO:1990045] Definition: Any process that stops, prevents or reduces the frequency, rate or extent of sclerotium development. Also known as: down regulation of sclerotium development, down-regulation of sclerotium development, downregulation of sclerotium development, inhibition of sclerotium development References: PMID:21148914 Sources: GOC:TermGenie, GOC:di